{
  "term_label": "positive regulation of canonical Wnt signaling pathway",
  "gene_symbol": "NRARP",
  "term_id": "GO:0090263",
  "gene_name": "Notch-regulated ankyrin repeat-containing protein",
  "gene": "UniProtKB:Q7Z6K4"
}